{
  "gene_symbol": "EFS",
  "gene_name": "Embryonal Fyn-associated substrate",
  "term_label": "cytoplasm",
  "gene": "UniProtKB:O43281",
  "term_id": "GO:0005737"
}